{
  "term_id": "GO:0003755",
  "gene": "UniProtKB:P23284",
  "gene_symbol": "PPIB",
  "gene_name": "Peptidyl-prolyl cis-trans isomerase B",
  "term_label": "peptidyl-prolyl cis-trans isomerase activity"
}